{
  "term_id": "UNKNOWN:0001",
  "gene_name": "Ubiquitin carboxyl-terminal hydrolase 49",
  "gene": "UniProtKB:Q70CQ1",
  "gene_symbol": "USP49",
  "term_label": "Unknown molecular function"
}